{
  "gene_symbol": "NMS",
  "term_id": "UNKNOWN:0003",
  "gene": "UniProtKB:Q5H8A3",
  "gene_name": "Neuromedin-S",
  "term_label": "Unknown cellular component"
}